{
  "term_id": "GO:0006405",
  "gene_symbol": "NUP155",
  "term_label": "RNA export from nucleus",
  "gene": "UniProtKB:O75694",
  "gene_name": "Nuclear pore complex protein Nup155"
}